{
  "gene": "UniProtKB:O15528",
  "gene_symbol": "CYP27B1",
  "gene_name": "25-hydroxyvitamin D-1 alpha hydroxylase, mitochondrial",
  "term_label": "vitamin D catabolic process",
  "term_id": "GO:0042369"
}